{
  "gene": "UniProtKB:Q9UJU6",
  "term_label": "membrane organization",
  "gene_name": "Drebrin-like protein",
  "gene_symbol": "DBNL",
  "term_id": "GO:0061024"
}